negative regulation of type II hypersensitivity [GO:0002893] (biological process) Sources: GOC:add Subtypes: negative regulation of type IIa hypersensitivity [GO:0001797], negative regulation of type IIb hypersensitivity [GO:0001800] Also known as: down regulation of type II hypersensitivity, down-regulation of type II hypersensitivity, downregulation of type II hypersensitivity, inhibition of type II hypersensitivity Definition: Any process that stops, prevents, or reduces the frequency, rate, or extent of type II hypersensitivity. Relationships: is a type of negative regulation of hypersensitivity [GO:0002884]; is_a negative regulation of myeloid leukocyte mediated immunity [GO:0002887]; is a type of GO:0002890; is a type of regulation of type II hypersensitivity [GO:0002892]; negatively regulates GO:0002445